{
  "gene_symbol": "OR6T1",
  "gene_name": "Olfactory receptor 6T1",
  "gene": "UniProtKB:Q8NGN1",
  "term_id": "UNKNOWN:0002",
  "term_label": "Unknown biological process"
}